{
  "term_label": "nucleus",
  "gene_symbol": "RBP1",
  "gene": "UniProtKB:P09455",
  "term_id": "GO:0005634",
  "gene_name": "Retinol-binding protein 1"
}